{
  "gene": "UniProtKB:Q969G2",
  "gene_name": "LIM_homeobox protein Lhx4",
  "term_id": "GO:0006357",
  "gene_symbol": "LHX4",
  "term_label": "regulation of transcription by RNA polymerase II"
}